glucan 1,6-alpha-isomaltosidase activity [GO:0033923] (molecular function) Also known as: 1,6-alpha-D-glucan isomaltohydrolase activity, G2-dextranase activity, exo-isomaltohydrolase activity, isomalto-dextranase activity, isomaltodextranase activity Sources: EC:3.2.1.94 Definition: Catalysis of the hydrolysis of (1->6)-alpha-D-glucosidic linkages in polysaccharides, to remove successive isomaltose units from the non-reducing ends of the chains. Relationships: is a type of hydrolase activity, hydrolyzing O-glycosyl compounds [GO:0004553]